{
  "term_label": "actin binding",
  "term_id": "GO:0003779",
  "gene": "UniProtKB:Q9NVD7",
  "gene_name": "Alpha-parvin",
  "gene_symbol": "PARVA"
}